{
  "term_label": "oxygen carrier activity",
  "term_id": "GO:0005344",
  "gene": "UniProtKB:P69905",
  "gene_symbol": "HBA2",
  "gene_name": "Hemoglobin subunit alpha"
}